positive regulation of L-tryptophan metabolic process [GO:0090358] (biological process) Definition: Any process that increases the frequency, rate or extent of the chemical reactions and pathways involving tryptophan, the chiral amino acid 2-amino-3-(1H-indol-3-yl)propanoic acid. Subtypes: positive regulation of 'de novo' NAD biosynthetic process from L-tryptophan [GO:1905014] Also known as: positive regulation of tryptophan metabolism, positive regulation of tryptophan metabolic process Sources: GOC:tb Relationships: is a type of positive regulation of amino acid metabolic process [GO:0045764]; is a type of positive regulation of small molecule metabolic process [GO:0062013]; is a type of regulation of L-tryptophan metabolic process [GO:0090357]; positively regulates GO:0006568